cerebellar Purkinje cell differentiation [GO:0021702] (biological process) Relationships: is a type of cell differentiation in hindbrain [GO:0021533]; is a type of central nervous system neuron differentiation [GO:0021953]; is part of cerebellar Purkinje cell layer formation [GO:0021694] Definition: The process in which neuroblasts acquire specialized structural and/or functional features that characterize the mature cerebellar Purkinje cell. Differentiation includes the processes involved in commitment of a neuroblast to a Purkinje cell fate. A Purkinje cell is an inhibitory GABAergic neuron found in the cerebellar cortex that projects to the deep cerebellar nuclei and brain stem. References: PMID:15157725 Sources: GOC:cls, GOC:dgh, GOC:dph, GOC:jid, GO_REF:0000021